inositol biosynthetic process [GO:0006021] (biological process) Regulation: regulated by regulation of inositol biosynthetic process [GO:1900088]; negatively regulated by GO:1900089; positively regulated by positive regulation of inositol biosynthetic process [GO:1900090] Also known as: inositol anabolism, inositol biosynthesis, inositol formation, inositol synthesis, vitamin Bh biosynthesis, vitamin Bh biosynthetic process, myo-inositol biosynthesis, myo-inositol biosynthetic process Sources: ISBN:0198547684 Relationships: is a type of GO:0006020; is a type of GO:0046173 Definition: The chemical reactions and pathways resulting in the formation of inositol, 1,2,3,4,5,6-cyclohexanehexol, a growth factor for animals and microorganisms.